{
  "term_label": "Unknown biological process",
  "gene_name": "HIRA-interacting protein 3",
  "term_id": "UNKNOWN:0002",
  "gene_symbol": "HIRIP3",
  "gene": "UniProtKB:Q9BW71"
}